{
  "gene": "UniProtKB:A0A3B3IS91",
  "gene_name": "POLG alternative reading frame",
  "gene_symbol": "POLGARF",
  "term_label": "Unknown molecular function",
  "term_id": "UNKNOWN:0001"
}